{
  "gene_symbol": "FGF5",
  "gene_name": "Fibroblast growth factor 5",
  "term_label": "cytoplasm",
  "gene": "UniProtKB:P12034",
  "term_id": "GO:0005737"
}